{
  "gene_symbol": "YBX1",
  "term_label": "regulation of gene expression",
  "gene": "UniProtKB:P67809",
  "gene_name": "Y-box-binding protein 1",
  "term_id": "GO:0010468"
}